{
  "term_id": "GO:0000175",
  "gene_name": "ERI1 exoribonuclease 3",
  "gene": "UniProtKB:O43414",
  "gene_symbol": "ERI3",
  "term_label": "3'-5'-RNA exonuclease activity"
}